{
  "term_label": "nucleus",
  "gene_name": "DnaJ homolog subfamily B member 8",
  "gene_symbol": "DNAJB8",
  "term_id": "GO:0005634",
  "gene": "UniProtKB:Q8NHS0"
}